{
  "term_label": "glomerulus development",
  "gene_symbol": "MYO1E",
  "gene_name": "Unconventional myosin-Ie",
  "term_id": "GO:0032835",
  "gene": "UniProtKB:Q12965"
}